{
  "gene": "UniProtKB:Q9P0J6",
  "gene_symbol": "MRPL36",
  "term_id": "GO:0005762",
  "gene_name": "Large ribosomal subunit protein bL36m",
  "term_label": "mitochondrial large ribosomal subunit"
}